tryptophanase activity [GO:0009034] (molecular function) Definition: Catalysis of the reaction: L-tryptophan + H2O = indole + NH4 + pyruvate. Relationships: is a type of GO:0016830; is part of L-tryptophan catabolic process [GO:0006569] Sources: RHEA:19553 Note: Note that this term has a MetaCyc pathway reference as the pathway only has a single step. Also known as: L-tryptophan indole-lyase (deaminating) activity, L-tryptophan indole-lyase (deaminating; pyruvate forming) activity, L-tryptophan indole-lyase activity, L-tryptophanase activity, TNase activity, tryptophan catabolic process, using tryptophanase, tryptophan catabolism, using tryptophanase